{
  "term_id": "GO:0004672",
  "term_label": "protein kinase activity",
  "gene_symbol": "NRK",
  "gene": "UniProtKB:Q7Z2Y5",
  "gene_name": "Nik-related protein kinase"
}